{
  "term_label": "RNA polymerase II cis-regulatory region sequence-specific DNA binding",
  "gene_name": "Zinc finger protein 628",
  "gene_symbol": "ZNF628",
  "gene": "UniProtKB:Q5EBL2",
  "term_id": "GO:0000978"
}